{
  "gene": "UniProtKB:P78368",
  "term_id": "GO:0005634",
  "gene_name": "Casein kinase I isoform gamma-2",
  "term_label": "nucleus",
  "gene_symbol": "CSNK1G2"
}